23S rRNA pseudouridine(2457) synthase activity [GO:0160137] (molecular function) Definition: Catalysis of the reaction: uridine(2457) in 23S rRNA = pseudouridine(2457) in 23S rRNA. Relationships: is_a GO:0120159 Sources: EC:5.4.99.20, RHEA:38871